{
  "gene_name": "Baculoviral IAP repeat-containing protein 7",
  "term_label": "regulation of cell cycle",
  "gene": "UniProtKB:Q96CA5",
  "term_id": "GO:0051726",
  "gene_symbol": "BIRC7"
}